{
  "term_id": "GO:0048013",
  "gene_symbol": "NCK2",
  "gene": "UniProtKB:O43639",
  "term_label": "ephrin receptor signaling pathway",
  "gene_name": "Cytoplasmic protein NCK2"
}